{
  "gene": "UniProtKB:P61106",
  "gene_symbol": "RAB14",
  "term_id": "GO:0006886",
  "gene_name": "Ras-related protein Rab-14",
  "term_label": "intracellular protein transport"
}